regulation of branching involved in salivary gland morphogenesis by mesenchymal-epithelial signaling [GO:0060665] (BP) Relationships: is a type of mesenchymal-epithelial cell signaling [GO:0060638]; is a type of regulation of branching involved in salivary gland morphogenesis [GO:0060693] Also known as: regulation of branching involved in salivary gland morphogenesis by mesenchymal-epithelial signalling Definition: Any process that modulates the rate, frequency, or extent of branching involved in salivary gland morphogenesis as a result of signals being generated by the mesenchyme and received and interpreted by the salivary gland epithelium. References: PMID:17336109 Sources: GOC:dph